{
  "term_label": "Unknown molecular function",
  "gene_symbol": "TPRKB",
  "gene_name": "EKC_KEOPS complex subunit TPRKB",
  "term_id": "UNKNOWN:0001",
  "gene": "UniProtKB:Q9Y3C4"
}